{
  "term_id": "GO:0006888",
  "term_label": "endoplasmic reticulum to Golgi vesicle-mediated transport",
  "gene_name": "Transmembrane emp24 domain-containing protein 6",
  "gene": "UniProtKB:Q8WW62",
  "gene_symbol": "TMED6"
}